{
  "gene_name": "Rho guanine nucleotide exchange factor 9",
  "gene": "UniProtKB:O43307",
  "term_label": "postsynaptic specialization",
  "term_id": "GO:0099572",
  "gene_symbol": "ARHGEF9"
}